{
  "gene": "UniProtKB:Q9BYR8",
  "term_id": "UNKNOWN:0002",
  "term_label": "Unknown biological process",
  "gene_name": "Keratin-associated protein 3-1",
  "gene_symbol": "KRTAP3-1"
}